{
  "gene_symbol": "PTDSS1",
  "gene": "UniProtKB:P48651",
  "gene_name": "Phosphatidylserine synthase 1",
  "term_label": "Unknown biological process",
  "term_id": "UNKNOWN:0002"
}